{
  "term_label": "homogentisate catabolic process",
  "gene_name": "Fumarylacetoacetase",
  "gene": "UniProtKB:P16930",
  "gene_symbol": "FAH",
  "term_id": "GO:1902000"
}